{
  "gene": "UniProtKB:Q9P267",
  "gene_symbol": "MBD5",
  "term_label": "Unknown biological process",
  "term_id": "UNKNOWN:0002",
  "gene_name": "Methyl-CpG-binding domain protein 5"
}